6-hydroxycineole catabolic process [GO:0019639] (biological process) Sources: GOC:ai Also known as: 6-endo-hydroxycineole catabolic process, 6-endo-hydroxycineole catabolism, 6-hydroxycineole breakdown, 6-hydroxycineole catabolism, 6-hydroxycineole degradation, hydroxycineol catabolic process, hydroxycineol catabolism Relationships: is a type of monoterpenoid catabolic process [GO:0016100]; is a type of xenobiotic catabolic process [GO:0042178]; is a type of epoxide metabolic process [GO:0097176]; is a type of ether catabolic process [GO:1901502] Definition: The chemical reactions and pathways resulting in the breakdown of 6-hydroxycineole (6-hydroxy-1,8-epoxy-p-menthane), a hydrocarbon with the formula C10H18O2.